{
  "term_id": "UNKNOWN:0001",
  "gene": "UniProtKB:O75427",
  "gene_symbol": "LRCH4",
  "term_label": "Unknown molecular function",
  "gene_name": "Leucine-rich repeat and calponin homology domain-containing protein 4"
}